telomere maintenance via telomerase [GO:0007004] (biological process) Definition: The maintenance of proper telomeric length by the addition of telomeric repeats by telomerase. Also known as: telomerase-dependent telomere maintenance Sources: GOC:elh Relationships: is a type of RNA-templated DNA biosynthetic process [GO:0006278]; is a type of telomere maintenance via telomere lengthening [GO:0010833]; has part telomerase activity [GO:0003720]; has part telomere-telomerase complex assembly [GO:1905324] Regulation: regulated by regulation of telomere maintenance via telomerase [GO:0032210]; negatively regulated by negative regulation of telomere maintenance via telomerase [GO:0032211]; positively regulated by positive regulation of telomere maintenance via telomerase [GO:0032212]